{
  "term_id": "GO:0007399",
  "term_label": "nervous system development",
  "gene": "UniProtKB:O75581",
  "gene_name": "Low-density lipoprotein receptor-related protein 6",
  "gene_symbol": "LRP6"
}